silicic acid import across plasma membrane [GO:0015708] (biological process) Relationships: is_a GO:0098658 Also known as: silicate transport, silicic acid transport, silicic acid import, silicon uptake References: PMID:16572174 Sources: GOC:ai, GOC:krc Definition: The directed movement of silicates from outside of a cell, across the plasma membrane and into the cytosol. Silicates are the salts of silicic acids, and are usually composed of silicon and oxygen (Si[x]O[y]), one or more metals, and possibly hydrogen. Types of silicate include unisilicates, metasilicates and hydrous silicates.